{
  "term_label": "regulation of alternative mRNA splicing, via spliceosome",
  "gene": "UniProtKB:P49756",
  "gene_name": "RNA-binding protein 25",
  "gene_symbol": "RBM25",
  "term_id": "GO:0000381"
}